{
  "term_label": "BLOC-1 complex",
  "gene": "UniProtKB:Q6QNY0",
  "gene_name": "Biogenesis of lysosome-related organelles complex 1 subunit 3",
  "term_id": "GO:0031083",
  "gene_symbol": "BLOC1S3"
}